{
  "term_id": "GO:0016342",
  "term_label": "catenin complex",
  "gene": "UniProtKB:P35221",
  "gene_name": "Catenin alpha-1",
  "gene_symbol": "CTNNA1"
}